{
  "gene_symbol": "CA10",
  "term_id": "GO:0016836",
  "gene": "UniProtKB:Q9NS85",
  "gene_name": "Carbonic anhydrase-related protein 10",
  "term_label": "hydro-lyase activity"
}